{
  "term_label": "axon guidance",
  "gene_symbol": "PTPRO",
  "gene_name": "Receptor-type tyrosine-protein phosphatase O",
  "term_id": "GO:0007411",
  "gene": "UniProtKB:Q16827"
}